membrane depolarization [GO:0051899] (biological process) Definition: The process in which membrane potential decreases with respect to its steady-state potential, usually from negative potential to a more positive potential. For example, the initial depolarization during the rising phase of an action potential is in the direction from the negative steady-state resting potential towards the positive membrane potential that will be the peak of the action potential. Sources: GOC:dh, Wikipedia:Depolarization Relationships: is a type of regulation of membrane potential [GO:0042391] Regulation: regulated by regulation of membrane depolarization [GO:0003254]; negatively regulated by negative regulation of membrane depolarization [GO:1904180]; positively regulated by GO:1904181 Subtypes: mitochondrial depolarization [GO:0051882], GO:0086010, GO:1990736